{
  "term_id": "UNKNOWN:0003",
  "gene_name": "Nucleoporin-62 C-terminal-like protein",
  "gene_symbol": "NUP62CL",
  "term_label": "Unknown cellular component",
  "gene": "UniProtKB:Q9H1M0"
}